{
  "gene_symbol": "C15orf32",
  "term_label": "Unknown biological process",
  "term_id": "UNKNOWN:0002",
  "gene": "UniProtKB:Q32M92",
  "gene_name": "Uncharacterized protein C15orf32"
}